anterograde neuronal dense core vesicle transport [GO:1990048] (biological process) Regulation: regulated by regulation of anterograde dense core granule transport [GO:1901951]; negatively regulated by GO:1901952; positively regulated by positive regulation of anterograde dense core granule transport [GO:1901953] Relationships: is a type of anterograde axonal transport [GO:0008089]; is a type of vesicle transport along microtubule [GO:0047496]; is_a dense core granule cytoskeletal transport [GO:0099519] Also known as: anterograde dense core granule trafficking, anterograde dense core granule transport References: PMID:23358451 Sources: GOC:kmv Definition: The directed movement of substances in neuronal dense core vesicles along axonal microtubules towards the presynapse.